{
  "term_label": "adenylosuccinate synthase activity",
  "gene_symbol": "ADSS2",
  "gene_name": "Adenylosuccinate synthetase isozyme 2",
  "term_id": "GO:0004019",
  "gene": "UniProtKB:P30520"
}